{
  "term_label": "skeletal muscle contraction",
  "gene": "UniProtKB:P19237",
  "gene_symbol": "TNNI1",
  "term_id": "GO:0003009",
  "gene_name": "Troponin I, slow skeletal muscle"
}